{
  "term_label": "suppression of viral release by host",
  "gene_name": "E3 ubiquitin-protein ligase TRIM11",
  "gene_symbol": "TRIM11",
  "gene": "UniProtKB:Q96F44",
  "term_id": "GO:0044790"
}